intraciliary transport particle B binding [GO:0120170] (molecular function) Definition: Binding to an intraciliary transport particle B (IFT B) complex. Relationships: is a type of protein-containing complex binding [GO:0044877] Also known as: intraciliary transport complex B binding, intraflagellar transport complex B binding, intraflagellar transport particle B binding, IFT B complex binding References: PMID:20889716